cyclase activity [GO:0009975] (molecular function) Regulation: RO_0002211 by GO:0010851; negatively regulated by cyclase inhibitor activity [GO:0010852]; positively regulated by cyclase activator activity [GO:0010853]; positively regulated by positive regulation of cyclase activity [GO:0031281] Subtypes: RNA-3'-phosphate cyclase activity [GO:0003963], adenylate cyclase activity [GO:0004016], GO:0004383, tocopherol cyclase activity [GO:0009976], solanapyrone synthase activity [GO:0033190], GO:0034012, squalene cyclase activity [GO:0034072], halimadienyl-diphosphate synthase activity [GO:0035439], cyclic 2,3-diphosphoglycerate synthetase activity [GO:0036356], lycopene epsilon cyclase activity [GO:0045435], lycopene beta cyclase activity [GO:0045436], allene-oxide cyclase activity [GO:0046423], carboxy-cis,cis-muconate cyclase activity [GO:0047768], cytidylate cyclase activity [GO:0047805], GO:0047820, geranyl-diphosphate cyclase activity [GO:0047926], purine imidazole-ring cyclase activity [GO:0050230], sabinene synthase activity [GO:0080015], (-)-E-beta-caryophyllene synthase activity [GO:0080016], alpha-humulene synthase activity [GO:0080017] Sources: ISBN:0198547684 Definition: Catalysis of a ring closure reaction. Relationships: is a type of catalytic activity [GO:0003824]